GTPase activator activity [GO:0005096] (molecular function) Definition: Binds to and increases the activity of a GTPase, an enzyme that catalyzes the hydrolysis of GTP. Sources: GOC:mah Also known as: GAP activity, ARF GAP activity, ARF GTPase activator activity, Rab GAP activity, Rab GTPase activator activity, Rac GAP activity, Rac GTPase activator activity, Ral GAP activity, Ral GTPase activator activity, Ran GAP activity, Ran GTPase activator activity, RanGAP, Rap GAP activity, Rap GTPase activator activity, Ras GAP activity, Ras GTPase activator activity, Rho GAP activity, Rho GTPase activator activity, Sar GAP activity, Sar GTPase activator activity Note: Note that the name Sar derives from 'secretion-associated, Ras-related'. Relationships: is a type of enzyme activator activity [GO:0008047]; is a type of GO:0030695; positively regulates GTPase activity [GO:0003924]